{
  "gene_symbol": "TRBJ1-4",
  "gene_name": "T cell receptor beta joining 1-4",
  "term_label": "Unknown molecular function",
  "gene": "UniProtKB:A0A0J9YXG5",
  "term_id": "UNKNOWN:0001"
}